{
  "term_label": "positive chemotaxis",
  "term_id": "GO:0050918",
  "gene_name": "Fibroblast growth factor 10",
  "gene": "UniProtKB:O15520",
  "gene_symbol": "FGF10"
}